{
  "gene_symbol": "ZNF860",
  "gene": "UniProtKB:A6NHJ4",
  "gene_name": "Zinc finger protein 860",
  "term_label": "DNA-binding transcription factor activity, RNA polymerase II-specific",
  "term_id": "GO:0000981"
}